{
  "gene_symbol": "CCDC88A",
  "gene": "UniProtKB:Q3V6T2",
  "gene_name": "Girdin",
  "term_label": "cytoplasmic microtubule organization",
  "term_id": "GO:0031122"
}